{
  "term_id": "GO:0005886",
  "gene_symbol": "MAS1L",
  "gene": "UniProtKB:P35410",
  "term_label": "plasma membrane",
  "gene_name": "Mas-related G-protein coupled receptor MRG"
}